female sex determination [GO:0030237] (biological process) Definition: The specification of female sex of an individual organism. Subtypes: female germ-line sex determination [GO:0019099], female somatic sex determination [GO:0019101] Sources: GOC:mah, ISBN:0198506732 Relationships: is a type of sex determination [GO:0007530]; is part of GO:0007275